mycodextranase activity [GO:0033911] (molecular function) Relationships: is a type of hydrolase activity, hydrolyzing O-glycosyl compounds [GO:0004553] Sources: EC:3.2.1.61 Definition: Catalysis of the endohydrolysis of 1,4-alpha-D-glucosidic linkages in alpha-D-glucans containing both 1,3- and 1,4-bonds. Also known as: 1,3-1,4-alpha-D-glucan 4-glucanohydrolase activity